{
  "term_id": "GO:0051383",
  "gene_symbol": "NUF2",
  "gene": "UniProtKB:Q9BZD4",
  "term_label": "kinetochore organization",
  "gene_name": "Kinetochore protein Nuf2"
}